protein K33-linked ubiquitination [GO:1990390] (biological process) Definition: A protein ubiquitination process in which a polymer of ubiquitin, formed by linkages between lysine residues at position 33 of the ubiquitin monomers, is added to a protein. Relationships: is a type of protein polyubiquitination [GO:0000209] References: PMID:24768539